polysaccharide digestion [GO:0044245] (biological process) Relationships: is a type of digestion [GO:0007586] Sources: GOC:go_curators Definition: The whole of the physical, chemical, and biochemical processes carried out by living organisms to break down ingested polysaccharides into components that may be easily absorbed and directed into metabolism.